{
  "term_id": "GO:0005737",
  "gene": "UniProtKB:O94762",
  "gene_name": "ATP-dependent DNA helicase Q5",
  "term_label": "cytoplasm",
  "gene_symbol": "RECQL5"
}